{
  "term_label": "anatomical structure morphogenesis",
  "gene": "UniProtKB:Q99717",
  "term_id": "GO:0009653",
  "gene_symbol": "SMAD5",
  "gene_name": "Mothers against decapentaplegic homolog 5"
}